{
  "gene": "UniProtKB:Q96KX2",
  "gene_name": "F-actin-capping protein subunit alpha-3",
  "gene_symbol": "CAPZA3",
  "term_id": "GO:0008290",
  "term_label": "F-actin capping protein complex"
}